{
  "gene_name": "Uncharacterized protein",
  "term_label": "Unknown cellular component",
  "gene_symbol": "A0A2R8Y556",
  "gene": "UniProtKB:A0A2R8Y556",
  "term_id": "UNKNOWN:0003"
}